{
  "gene_name": "Putative FXYD domain-containing ion transport regulator 8",
  "gene": "UniProtKB:P58550",
  "gene_symbol": "FXYD6P3",
  "term_label": "Unknown cellular component",
  "term_id": "UNKNOWN:0003"
}